positive regulation of vasculogenesis [GO:2001214] (biological process) Relationships: is a type of positive regulation of cell differentiation [GO:0045597]; is_a regulation of vasculogenesis [GO:2001212]; positively regulates vasculogenesis [GO:0001570] Sources: GOC:obol Definition: Any process that activates or increases the frequency, rate or extent of vasculogenesis. Also known as: positive regulation of vascular morphogenesis